{
  "term_label": "protein phosphatase binding",
  "gene": "UniProtKB:P33151",
  "gene_name": "Cadherin-5",
  "gene_symbol": "CDH5",
  "term_id": "GO:0019903"
}